{
  "term_id": "GO:0005085",
  "gene_name": "Puratrophin-1",
  "gene": "UniProtKB:Q58EX7",
  "gene_symbol": "PLEKHG4",
  "term_label": "guanyl-nucleotide exchange factor activity"
}